{
  "term_label": "protein processing",
  "gene_name": "Presenilin-1",
  "gene_symbol": "PSEN1",
  "term_id": "GO:0016485",
  "gene": "UniProtKB:P49768"
}